arachidonate 14,15-epoxygenase activity [GO:0008404] (molecular function) Definition: Catalysis of an NADPH- and oxygen-dependent reaction that converts arachidonic acid to cis-14,15-epoxyeicosatrienoic acid. References: PMID:10681399 Sources: RHEA:51472, http://lipidlibrary.aocs.org/Lipids/eic_hete/index.htm Also known as: arachidonic acid 14,15-epoxygenase activity, cytochrome P450 CYP2C29, cytochrome P450 CYP2C39 Relationships: is a type of arachidonate epoxygenase activity [GO:0008392]